{
  "gene_name": "KRR1 small subunit processome component homolog",
  "term_id": "GO:0005730",
  "term_label": "nucleolus",
  "gene": "UniProtKB:Q13601",
  "gene_symbol": "KRR1"
}